hydrogen dehydrogenase (NADP+) activity [GO:0050583] (molecular function) Also known as: NADP-linked hydrogenase activity, NADP-reducing hydrogenase activity, hydrogen:NADP+ oxidoreductase activity Relationships: is a type of oxidoreductase activity, acting on hydrogen as donor, NAD or NADP as acceptor [GO:0016696] Sources: EC:1.12.1.3, MetaCyc:1.12.1.3-RXN Definition: Catalysis of the reaction: NADP+ + H2 = NADPH + H+.